cell body fiber [GO:0070852] (CC) Sources: GOC:dos, GOC:mah Relationships: is a type of neuron projection [GO:0043005] Definition: A neuron projection that is found in unipolar neurons and corresponds to the region between the cell body and the point at which the single projection branches. Also known as: cell body fibre, primary neurite